actin ubiquitination [GO:0007014] (biological process) Also known as: indirect flight muscle actin ubiquitination Definition: The modification of actin by addition of ubiquitin groups. Sources: GOC:mah Relationships: is a type of protein ubiquitination [GO:0016567]; is a type of GO:0030047